{
  "gene": "UniProtKB:Q96BT1",
  "gene_symbol": "C3orf49",
  "term_id": "UNKNOWN:0002",
  "gene_name": "Putative uncharacterized protein C3orf49",
  "term_label": "Unknown biological process"
}